ethylene catabolic process [GO:0042457] (biological process) Definition: The chemical reactions and pathways resulting in the breakdown of ethylene (C2-H4, ethene), a simple hydrocarbon gas that can function in plants as a growth regulator. Sources: GOC:jl, ISBN:0387969845 Also known as: ethene catabolic process, ethene catabolism, ethylene breakdown, ethylene catabolism, ethylene degradation Relationships: is a type of GO:0009692; is a type of alkene catabolic process [GO:0043451]